response to aromatase inhibitor [GO:0061477] (biological process) Sources: GOC:dph Definition: Any process that results in a change in state or activity of a cell or an organism (in terms of movement, secretion, enzyme production, gene expression, etc.) as a result of an aromatase inhibitor stimulus. Relationships: is a type of response to chemical [GO:0042221]